{
  "term_id": "UNKNOWN:0001",
  "gene_name": "T-complex protein 11 X-linked protein 1",
  "gene": "UniProtKB:B4DZS4",
  "term_label": "Unknown molecular function",
  "gene_symbol": "TCP11X1"
}